{
  "term_label": "cytoplasmic stress granule",
  "gene_name": "Lupus La protein",
  "gene_symbol": "SSB",
  "gene": "UniProtKB:P05455",
  "term_id": "GO:0010494"
}